{
  "term_label": "phosphopyruvate hydratase activity",
  "gene": "UniProtKB:P13929",
  "gene_name": "Beta-enolase",
  "gene_symbol": "ENO3",
  "term_id": "GO:0004634"
}